protein-lysine-acetyltransferase activity [GO:0061733] (molecular function) Definition: Catalysis of the reaction: L-lysyl-[protein] + acetyl-CoA = N6-acetyl-L-lysyl-[protein] + CoA + H+. Sources: RHEA:45948 Also known as: protein acetylase activity, protein acetyltransferase activity, peptide-lysine-N-acetylase activity, peptide-lysine-N-acetyltransferase activity, peptide-lysine-acetyltransferase activity, protein-lysine-N-acetylase activity Relationships: is_a GO:0034212 Subtypes: histone acetyltransferase activity [GO:0004402], GO:0019799